{
  "term_label": "cytoplasm",
  "gene": "UniProtKB:Q16829",
  "term_id": "GO:0005737",
  "gene_name": "Dual specificity protein phosphatase 7",
  "gene_symbol": "DUSP7"
}